{
  "gene_name": "G_T mismatch-specific thymine DNA glycosylase",
  "gene_symbol": "TDG",
  "term_id": "GO:0008263",
  "term_label": "pyrimidine-specific mismatch base pair DNA N-glycosylase activity",
  "gene": "UniProtKB:Q13569"
}